{
  "gene_name": "Salivary gland specific protein SAGSIN1",
  "term_id": "UNKNOWN:0002",
  "term_label": "Unknown biological process",
  "gene": "UniProtKB:A0A0C4DGP1",
  "gene_symbol": "SAGSIN1"
}